cellular response to retinoic acid [GO:0071300] (biological process) Definition: Any process that results in a change in state or activity of a cell (in terms of movement, secretion, enzyme production, gene expression, etc.) as a result of a retinoic acid stimulus. Sources: GOC:mah Also known as: cellular response to vitamin A acid Relationships: is a type of response to retinoic acid [GO:0032526]; is_a cellular response to lipid [GO:0071396]; is a type of cellular response to oxygen-containing compound [GO:1901701]